{
  "gene": "UniProtKB:Q9Y6Z5",
  "term_id": "UNKNOWN:0002",
  "term_label": "Unknown biological process",
  "gene_symbol": "AFDN-DT",
  "gene_name": "Putative uncharacterized protein AFDN-DT"
}